{
  "gene_name": "CMRF35-like molecule 2",
  "term_label": "plasma membrane",
  "gene_symbol": "CD300E",
  "gene": "UniProtKB:Q496F6",
  "term_id": "GO:0005886"
}